{
  "term_label": "endoplasmic reticulum",
  "gene_symbol": "FAF1",
  "term_id": "GO:0005783",
  "gene_name": "FAS-associated factor 1",
  "gene": "UniProtKB:Q9UNN5"
}